{
  "term_id": "GO:0047023",
  "gene_name": "Aldo-keto reductase family 1 member C1",
  "gene_symbol": "AKR1C1",
  "gene": "UniProtKB:Q04828",
  "term_label": "androsterone dehydrogenase [NAD(P)+] activity"
}